{
  "term_label": "Unknown molecular function",
  "gene": "UniProtKB:A0N4Z3",
  "gene_name": "HCG2039775 (Fragment)",
  "term_id": "UNKNOWN:0001",
  "gene_symbol": "TRAJ14"
}